{
  "gene": "UniProtKB:Q9P2D1",
  "gene_symbol": "CHD7",
  "term_label": "heart morphogenesis",
  "gene_name": "Chromodomain-helicase-DNA-binding protein 7",
  "term_id": "GO:0003007"
}